{
  "gene_symbol": "NAXE",
  "gene": "UniProtKB:Q8NCW5",
  "term_label": "NAD(P)HX epimerase activity",
  "gene_name": "NAD(P)H-hydrate epimerase",
  "term_id": "GO:0052856"
}